{
  "gene": "UniProtKB:P0DN25",
  "gene_name": "C1GALT1-specific chaperone 1-like protein",
  "term_label": "Unknown biological process",
  "term_id": "UNKNOWN:0002",
  "gene_symbol": "C1GALT1C1L"
}